{
  "gene_name": "LIM and senescent cell antigen-like-containing domain protein 1",
  "term_label": "cell-cell junction",
  "gene_symbol": "LIMS1",
  "gene": "UniProtKB:P48059",
  "term_id": "GO:0005911"
}